 [oboInOwl#is:metadata:tag]